isomaltulose synthase activity [GO:0050006] (MF) Sources: EC:5.4.99.11, MetaCyc:ISOMALTULOSE-SYNTHASE-RXN Relationships: is a type of intramolecular transferase activity [GO:0016866] Definition: Catalysis of the reaction: sucrose = 6-O-alpha-D-glucopyranosyl-D-fructofuranose. Also known as: isomaltulose synthetase activity, sucrose alpha-glucosyltransferase activity, sucrose glucosylmutase activity, trehalulose synthase activity